{
  "term_label": "RNA polymerase II cis-regulatory region sequence-specific DNA binding",
  "gene": "UniProtKB:P78413",
  "term_id": "GO:0000978",
  "gene_symbol": "IRX4",
  "gene_name": "Iroquois-class homeodomain protein IRX-4"
}